{
  "term_label": "G protein-coupled bile acid receptor activity",
  "gene": "UniProtKB:Q8TDU6",
  "term_id": "GO:0038182",
  "gene_symbol": "GPBAR1",
  "gene_name": "G-protein coupled bile acid receptor 1"
}